negative regulation of convergent extension involved in rhombomere morphogenesis [GO:1904134] (BP) References: PMID:24892953 Sources: GOC:TermGenie, GOC:dph, GO_REF:0000058 Also known as: down regulation of convergent extension involved in rhombomere morphogenesis, down-regulation of convergent extension involved in rhombomere morphogenesis, downregulation of convergent extension involved in rhombomere morphogenesis, inhibition of convergent extension involved in rhombomere morphogenesis Relationships: is_a GO:1904104; is_a GO:1904133; negatively regulates GO:1904125 Definition: Any process that stops, prevents or reduces the frequency, rate or extent of convergent extension involved in rhombomere morphogenesis.